{
  "gene_symbol": "MSX2",
  "term_label": "nucleus",
  "term_id": "GO:0005634",
  "gene_name": "Homeobox protein MSX-2",
  "gene": "UniProtKB:P35548"
}